{
  "gene_symbol": "CNTNAP5",
  "term_label": "plasma membrane",
  "gene_name": "Contactin-associated protein-like 5",
  "gene": "UniProtKB:Q8WYK1",
  "term_id": "GO:0005886"
}